{
  "term_label": "excitatory extracellular ligand-gated monoatomic ion channel activity",
  "gene_symbol": "GLRA2",
  "gene_name": "Glycine receptor subunit alpha-2",
  "term_id": "GO:0005231",
  "gene": "UniProtKB:P23416"
}